response to muscle activity [GO:0014850] (biological process) Sources: GOC:mtg_muscle Definition: Any process that results in a change in state or activity of a cell or an organism (in terms of movement, secretion, enzyme production, gene expression, etc.) as a result of a muscle activity stimulus. Subtypes: detection of muscle activity [GO:0014864], GO:0014873 Relationships: is_a GO:0014823